{
  "gene_symbol": "A8MVJ9",
  "term_id": "GO:0005634",
  "gene_name": "Putative histone PARylation factor 1-like",
  "term_label": "nucleus",
  "gene": "UniProtKB:A8MVJ9"
}